ARF protein signal transduction [GO:0032011] (biological process) Sources: GOC:mah Regulation: RO_0002211 by GO:0032012; negatively regulated by GO:0032013; positively regulated by positive regulation of ARF protein signal transduction [GO:0032014] Definition: An intracellular signaling cassette in which a small monomeric GTPase of the ARF subfamily relays a signal. Relationships: is a type of small GTPase-mediated signal transduction [GO:0007264]